{
  "gene_symbol": "PDE1B",
  "gene": "UniProtKB:Q01064",
  "gene_name": "Dual specificity calcium_calmodulin-dependent 3',5'-cyclic nucleotide phosphodiesterase 1B",
  "term_label": "negative regulation of cAMP/PKA signal transduction",
  "term_id": "GO:0141162"
}